{
  "gene_symbol": "ARHGEF40",
  "gene_name": "Rho guanine nucleotide exchange factor 40",
  "term_label": "extrinsic component of membrane",
  "term_id": "GO:0019898",
  "gene": "UniProtKB:Q8TER5"
}